{
  "gene": "UniProtKB:O00194",
  "gene_symbol": "RAB27B",
  "term_label": "GTP binding",
  "term_id": "GO:0005525",
  "gene_name": "Ras-related protein Rab-27B"
}